{
  "gene_name": "Leucine-rich repeat-containing protein 23",
  "term_id": "GO:0030317",
  "gene_symbol": "LRRC23",
  "term_label": "flagellated sperm motility",
  "gene": "UniProtKB:Q53EV4"
}